{
  "term_id": "GO:0033389",
  "gene_symbol": "AGMAT",
  "gene": "UniProtKB:Q9BSE5",
  "gene_name": "Guanidino acid hydrolase, mitochondrial",
  "term_label": "putrescine biosynthetic process from arginine, via agmatine"
}